{
  "gene_symbol": "GSPT2",
  "gene_name": "Eukaryotic peptide chain release factor GTP-binding subunit ERF3B",
  "term_id": "GO:0003747",
  "gene": "UniProtKB:Q8IYD1",
  "term_label": "translation release factor activity"
}